{
  "term_id": "GO:0010468",
  "gene_name": "Ret finger protein-like 1",
  "term_label": "regulation of gene expression",
  "gene": "UniProtKB:O75677",
  "gene_symbol": "RFPL1"
}